{
  "term_label": "[methionine synthase] reductase (NADPH) activity",
  "gene_name": "Methionine synthase reductase",
  "gene": "UniProtKB:Q9UBK8",
  "gene_symbol": "MTRR",
  "term_id": "GO:0030586"
}